{
  "gene": "UniProtKB:Q96NY7",
  "term_label": "D3 dopamine receptor binding",
  "gene_name": "Chloride intracellular channel protein 6",
  "gene_symbol": "CLIC6",
  "term_id": "GO:0031750"
}